{
  "gene": "UniProtKB:Q9H320",
  "term_label": "Unknown cellular component",
  "term_id": "UNKNOWN:0003",
  "gene_symbol": "VCX",
  "gene_name": "Variable charge X-linked protein 1"
}